survivin complex [GO:1990713] (cellular component) Relationships: is a type of nuclear protein-containing complex [GO:0140513] Also known as: Baculoviral IAP repeat-containing protein 5 complex, survivin homodimer complex References: PMID:10949038 Sources: GOC:bhm Definition: A protein complex that negatively regulates apoptotic processes. In human, this anti-apoptotic complex is a homodimer of BIRC5 (survivin) and provides one survivin molecule to the chromosomal passenger complex (CPC). Note: An example of this is BIRC5 in human (UniProt symbol O15392) in PMID:10949038 (inferred from physical interaction).